{
  "gene": "UniProtKB:O60494",
  "gene_symbol": "CUBN",
  "gene_name": "Cubilin",
  "term_id": "GO:0005886",
  "term_label": "plasma membrane"
}